transport along microtubule [GO:0010970] (biological process) Subtypes: GO:0008088, intraciliary transport [GO:0042073], GO:0072384, protein transport along microtubule [GO:0098840] Sources: GOC:dph, GOC:mah, GOC:tb Definition: The movement of organelles or other particles from one location in the cell to another along microtubules, driven by motor activity. Also known as: microtubule-based transport, establishment of localization by movement along microtubule, movement along microtubule Relationships: is_a GO:0007018; is a type of cytoskeleton-dependent intracellular transport [GO:0030705]; is a type of microtubule-based transport [GO:0099111]